regulation of endocrine process [GO:0044060] (biological process) Sources: GOC:jl Definition: Any process that modulates the frequency, rate or extent of an endocrine process, a process involving the secretion of or response to endocrine hormones. An endocrine hormone is a hormone released into the circulatory system. Subtypes: regulation of juvenile hormone secretion [GO:0007558], GO:0032276, regulation of inhibin secretion [GO:0032338], regulation of corticotropin secretion [GO:0051459], GO:1900133, regulation of parathyroid hormone secretion [GO:2000828], GO:2000831 Also known as: regulation of endocrine system process Relationships: is a type of regulation of system process [GO:0044057]; regulates endocrine process [GO:0050886]